{
  "gene": "UniProtKB:Q9HB20",
  "gene_name": "Pleckstrin homology domain-containing family A member 3",
  "term_label": "endosome organization",
  "gene_symbol": "PLEKHA3",
  "term_id": "GO:0007032"
}